{
  "term_label": "selenocysteine incorporation",
  "term_id": "GO:0001514",
  "gene": "UniProtKB:P57772",
  "gene_name": "Selenocysteine-specific elongation factor",
  "gene_symbol": "EEFSEC"
}